{
  "term_id": "UNKNOWN:0002",
  "gene_name": "tRNA (guanine(10)-N2)-methyltransferase homolog",
  "gene_symbol": "TRMT11",
  "term_label": "Unknown biological process",
  "gene": "UniProtKB:Q7Z4G4"
}